{
  "gene_symbol": "OSGEP",
  "term_id": "UNKNOWN:0002",
  "gene": "UniProtKB:Q9NPF4",
  "term_label": "Unknown biological process",
  "gene_name": "tRNA N6-adenosine threonylcarbamoyltransferase"
}